{
  "gene": "UniProtKB:Q96RQ1",
  "term_label": "Unknown molecular function",
  "term_id": "UNKNOWN:0001",
  "gene_symbol": "ERGIC2",
  "gene_name": "Endoplasmic reticulum-Golgi intermediate compartment protein 2"
}